{
  "term_label": "antigen binding",
  "gene_name": "Immunoglobulin heavy variable 3-48",
  "gene": "UniProtKB:P01763",
  "term_id": "GO:0003823",
  "gene_symbol": "IGHV3-48"
}